Shu complex [GO:0097196] (cellular component) References: PMID:15654096, PMID:19496932 Sources: GOC:jh Relationships: is a type of protein-containing complex [GO:0032991] Definition: A protein complex involved in error-free DNA post-replication repair (PRR). In Saccharomyces cerevisiae the complex contains Csm2p, Psy3p, Shu1p, and Shu2p.